{
  "term_label": "Unknown molecular function",
  "gene_name": "Synaptic vesicle glycoprotein 2C",
  "gene_symbol": "SV2C",
  "term_id": "UNKNOWN:0001",
  "gene": "UniProtKB:Q496J9"
}